{
  "gene": "UniProtKB:P25101",
  "term_label": "endothelin receptor signaling pathway",
  "term_id": "GO:0086100",
  "gene_symbol": "EDNRA",
  "gene_name": "Endothelin-1 receptor"
}